{
  "gene": "UniProtKB:O95786",
  "term_id": "GO:0003725",
  "gene_name": "Antiviral innate immune response receptor RIG-I",
  "gene_symbol": "RIGI",
  "term_label": "double-stranded RNA binding"
}